positive regulation of uredospore formation [GO:0075253] (biological process) Definition: Any process that activates, maintains or increases the frequency, rate or extent of uredospore formation, a process in which an asexual, dikaryotic, often rusty-colored spore, is formed in a structure called a uredinium. Also known as: positive regulation of ureidospore formation Sources: GOC:pamgo_curators Relationships: is a type of GO:0043945; is a type of regulation of uredospore formation [GO:0075252]; positively regulates uredospore formation [GO:0075251]